{
  "term_id": "GO:0005634",
  "gene_symbol": "MDC1",
  "term_label": "nucleus",
  "gene_name": "Mediator of DNA damage checkpoint protein 1",
  "gene": "UniProtKB:Q14676"
}